{
  "gene_name": "Diphosphoinositol polyphosphate phosphohydrolase 3-beta",
  "gene_symbol": "NUDT11",
  "term_label": "diphosphoinositol-polyphosphate diphosphatase activity",
  "term_id": "GO:0008486",
  "gene": "UniProtKB:Q96G61"
}